rhythmic synaptic transmission [GO:0060024] (biological process) Relationships: is a type of modulation of chemical synaptic transmission [GO:0050804] Definition: Any process involved in the generation of rhythmic, synchronous synaptic inputs in a neural circuit. Subtypes: rhythmic excitation [GO:0043179], rhythmic inhibition [GO:0043180] Sources: GOC:dph